{
  "gene_symbol": "EEF1A1",
  "gene": "UniProtKB:P68104",
  "term_id": "UNKNOWN:0003",
  "term_label": "Unknown cellular component",
  "gene_name": "Elongation factor 1-alpha 1"
}